{
  "term_label": "nuclear pore central transport channel",
  "gene": "UniProtKB:Q9UKK6",
  "gene_symbol": "NXT1",
  "gene_name": "NTF2-related export protein 1",
  "term_id": "GO:0044613"
}